macrophage tolerance induction [GO:0010931] (biological process) Regulation: regulated by GO:0010932; positively regulated by positive regulation of macrophage tolerance induction [GO:0010933] Relationships: is a type of tolerance induction [GO:0002507] Sources: GOC:BHF, GOC:dph, GOC:tb Definition: A process involving any mechanism for tolerance induction in macrophages.